{
  "gene": "UniProtKB:P0C7T3",
  "gene_symbol": "OR56A5",
  "term_label": "olfactory receptor activity",
  "term_id": "GO:0004984",
  "gene_name": "Olfactory receptor 56A5"
}